{
  "term_label": "microtubule-based movement",
  "gene_name": "Kinesin-like protein KIF12",
  "gene_symbol": "KIF12",
  "term_id": "GO:0007018",
  "gene": "UniProtKB:Q96FN5"
}